{
  "term_label": "histone binding",
  "gene_symbol": "TSPY10",
  "gene": "UniProtKB:P0CW01",
  "term_id": "GO:0042393",
  "gene_name": "Testis-specific Y-encoded protein 10"
}